{
  "term_id": "GO:0043186",
  "gene_symbol": "DDX3X",
  "gene_name": "ATP-dependent RNA helicase DDX3X",
  "term_label": "P granule",
  "gene": "UniProtKB:O00571"
}